neutrophil apoptotic process [GO:0001781] (biological process) Definition: Any apoptotic process in a neutrophil, any of the immature or mature forms of a granular leukocyte that in its mature form has a nucleus with three to five lobes connected by slender threads of chromatin, and cytoplasm containing fine inconspicuous granules and stainable by neutral dyes. References: PMID:12752675, PMID:12960266 Sources: CL:0000775, GOC:add, GOC:mtg_apoptosis Also known as: apoptosis of neutrophils, neutrophil programmed cell death by apoptosis, programmed cell death of neutrophils by apoptosis, programmed cell death, neutrophils, neutrophil apoptosis Relationships: is_a inflammatory cell apoptotic process [GO:0006925]; is a type of myeloid cell apoptotic process [GO:0033028]; is a type of leukocyte apoptotic process [GO:0071887]; is part of neutrophil homeostasis [GO:0001780] Regulation: regulated by GO:0033029; negatively regulated by negative regulation of neutrophil apoptotic process [GO:0033030]; positively regulated by GO:0033031